{
  "gene_name": "Mitoferrin-2",
  "term_label": "iron import into the mitochondrion",
  "gene": "UniProtKB:Q96A46",
  "gene_symbol": "SLC25A28",
  "term_id": "GO:0048250"
}